ghrelin receptor binding [GO:0031768] (molecular function) Definition: Binding to a ghrelin receptor. Sources: GOC:mah, GOC:nln Relationships: is a type of G protein-coupled receptor binding [GO:0001664] Also known as: type 1 growth hormone secretagogue GH-releasing peptide receptor binding, ghrelin receptor ligand